{
  "gene_name": "Transmembrane protein 213",
  "term_id": "UNKNOWN:0002",
  "term_label": "Unknown biological process",
  "gene_symbol": "TMEM213",
  "gene": "UniProtKB:A2RRL7"
}